{
  "term_label": "protein retention in Golgi apparatus",
  "gene": "UniProtKB:Q92673",
  "term_id": "GO:0045053",
  "gene_name": "Sortilin-related receptor",
  "gene_symbol": "SORL1"
}